regulation of spermatid nuclear differentiation [GO:0045700] (biological process) Sources: GOC:go_curators Definition: Any process that modulates the frequency, rate or extent of spermatid nuclear differentiation. Subtypes: GO:0045701, positive regulation of spermatid nuclear differentiation [GO:0045702] Relationships: is a type of regulation of multicellular organismal process [GO:0051239]; is_a regulation of nucleus organization [GO:1903353]; regulates spermatid nucleus differentiation [GO:0007289]